{
  "gene_name": "Nuclear factor NF-kappa-B p100 subunit",
  "term_label": "RNA polymerase II cis-regulatory region sequence-specific DNA binding",
  "gene_symbol": "NFKB2",
  "gene": "UniProtKB:Q00653",
  "term_id": "GO:0000978"
}